{
  "gene_name": "Nanos homolog 1",
  "gene": "UniProtKB:Q8WY41",
  "term_label": "perinuclear region of cytoplasm",
  "term_id": "GO:0048471",
  "gene_symbol": "NANOS1"
}